glutaminase complex [GO:1903600] (cellular component) Definition: A protein complex which is capable of glutaminase activity. References: PMID:14764090 Sources: GOC:TermGenie, GO_REF:0000088 Also known as: Sno1p-Snz1p Relationships: is a type of catalytic complex [GO:1902494]